{
  "term_label": "carbohydrate metabolic process",
  "gene": "UniProtKB:P0DUB6",
  "term_id": "GO:0005975",
  "gene_name": "Alpha-amylase 1A",
  "gene_symbol": "AMY1A"
}